{
  "gene": "UniProtKB:Q96AQ7",
  "gene_symbol": "CIDEC",
  "gene_name": "Lipid transferase CIDEC",
  "term_label": "lipid storage",
  "term_id": "GO:0019915"
}